{
  "term_label": "plasma membrane",
  "gene": "UniProtKB:Q8TBJ4",
  "gene_name": "Phospholipid phosphatase-related protein type 1",
  "gene_symbol": "PLPPR1",
  "term_id": "GO:0005886"
}